{
  "gene_name": "CREB-regulated transcription coactivator 2",
  "term_id": "GO:0008140",
  "gene_symbol": "CRTC2",
  "term_label": "cAMP response element binding protein binding",
  "gene": "UniProtKB:Q53ET0"
}